pyridoxal phosphate catabolic process [GO:0032361] (BP) Relationships: is a type of GO:0042820; is a type of pyridoxal phosphate metabolic process [GO:0042822]; is a type of aldehyde catabolic process [GO:0046185]; is_a organophosphate catabolic process [GO:0046434] Definition: The chemical reactions and pathways resulting in the breakdown of pyridoxal phosphate, pyridoxal phosphorylated at the hydroxymethyl group of C-5, the active form of vitamin B6. Sources: GOC:mah